{
  "gene_name": "Partner and localizer of BRCA2",
  "gene": "UniProtKB:Q86YC2",
  "term_id": "GO:0005654",
  "gene_symbol": "PALB2",
  "term_label": "nucleoplasm"
}